{
  "gene_name": "Coiled-coil domain-containing protein 85A",
  "term_id": "UNKNOWN:0001",
  "gene": "UniProtKB:Q96PX6",
  "term_label": "Unknown molecular function",
  "gene_symbol": "CCDC85A"
}